{
  "gene_name": "Prolactin receptor",
  "gene": "UniProtKB:P16471",
  "term_id": "GO:0019955",
  "term_label": "cytokine binding",
  "gene_symbol": "PRLR"
}